{
  "term_label": "NuRD complex",
  "term_id": "GO:0016581",
  "gene_symbol": "HDAC1",
  "gene_name": "Histone deacetylase 1",
  "gene": "UniProtKB:Q13547"
}